amino acid catabolic process to carboxylic acid via Ehrlich pathway [GO:0000948] (biological process) Relationships: is a type of amino acid catabolic process via Ehrlich pathway [GO:0000955]; is a type of carboxylic acid biosynthetic process [GO:0046394] References: PMID:18281432 Sources: GOC:krc Definition: The chemical reactions and pathways involving the catabolism of amino acids to produce carboxylic acids with one carbon less than the starting amino acid. In S. cerevisiae, this is known to occur for leucine, isoleucine, valine, methionine, phenylalanine, tyrosine, or tryptophan. Often referred to as the Ehrlich pathway, these reactions generally occur during fermentation to produce a variety of carboxylic acids, sometimes collectively referred to as fusel acids. Depending on the redox state of the cells, alcohol derivatives may be produced instead of carboxylic acids. Subtypes: aromatic amino acid family catabolic process to carboxylic acid via Ehrlich pathway [GO:0000952], branched-chain amino acid catabolic process to carboxylic acid via Ehrlich pathway [GO:0000953], L-methionine catabolic process to 3-methylthiopropanoate [GO:0000954]